{
  "gene": "UniProtKB:A0A1Y8EI39",
  "gene_name": "Immunoglobulin heavy diversity 6-13 (Fragment)",
  "term_id": "UNKNOWN:0001",
  "term_label": "Unknown molecular function",
  "gene_symbol": "IGHD6-13"
}